{
  "gene_name": "G-protein coupled receptor 182",
  "term_id": "UNKNOWN:0003",
  "term_label": "Unknown cellular component",
  "gene_symbol": "GPR182",
  "gene": "UniProtKB:O15218"
}